{
  "gene_symbol": "KAT5",
  "term_label": "NuA4 histone acetyltransferase complex",
  "gene": "UniProtKB:Q92993",
  "gene_name": "Histone acetyltransferase KAT5",
  "term_id": "GO:0035267"
}